regulation of uredospore formation [GO:0075252] (biological process) Definition: Any process that modulates the frequency, rate or extent of uredospore formation, a process in which an asexual, dikaryotic, often rusty-colored spore, is formed in a structure called a uredinium. Sources: GOC:pamgo_curators Also known as: regulation of ureidospore formation Relationships: is a type of regulation of asexual sporulation resulting in formation of a cellular spore [GO:0043943]; RO_0002211 GO:0075251 Subtypes: positive regulation of uredospore formation [GO:0075253], negative regulation of uredospore formation [GO:0075254]